regulation of cell population proliferation [GO:0042127] (biological process) Definition: Any process that modulates the frequency, rate or extent of cell proliferation. Relationships: is a type of regulation of cellular process [GO:0050794]; regulates GO:0008283 Also known as: regulation of cell proliferation Subtypes: GO:0003420, positive regulation of cell population proliferation [GO:0008284], negative regulation of cell population proliferation [GO:0008285], regulation of mesenchymal cell proliferation [GO:0010464], GO:0014857, regulation of osteoblast proliferation [GO:0033688], GO:0035206, GO:0048145, regulation of smooth muscle cell proliferation [GO:0048660], regulation of epithelial cell proliferation [GO:0050678], regulation of cardiac muscle cell proliferation [GO:0060043], GO:0060251, regulation of cell proliferation involved in embryonic placenta development [GO:0060723], regulation of cell proliferation involved in tissue homeostasis [GO:0060784], regulation of cell proliferation involved in kidney morphogenesis [GO:0061006], regulation of fat cell proliferation [GO:0070344], regulation of leukocyte proliferation [GO:0070663], regulation of hair follicle cell proliferation [GO:0071336], regulation of cell proliferation in bone marrow [GO:0071863], regulation of stem cell proliferation [GO:0072091], regulation of cell proliferation involved in imaginal disc-derived wing morphogenesis [GO:0090256], regulation of chorionic trophoblast cell proliferation [GO:1901382], regulation of cell proliferation involved in kidney development [GO:1901722], GO:1904073, regulation of germ cell proliferation [GO:1905936], regulation of mammary stem cell proliferation [GO:2000101], regulation of cell proliferation involved in heart morphogenesis [GO:2000136], regulation of neural precursor cell proliferation [GO:2000177], regulation of myoblast proliferation [GO:2000291], GO:2000495 Sources: GOC:jl